citrulline metabolic process [GO:0000052] (biological process) Definition: The chemical reactions and pathways involving citrulline, N5-carbamoyl-L-ornithine, an alpha amino acid not found in proteins. Subtypes: citrulline biosynthetic process [GO:0019240], L-citrulline catabolic process [GO:0019241] Sources: ISBN:0198506732 Relationships: is_a non-proteinogenic amino acid metabolic process [GO:0170041]; is a type of alpha-amino acid metabolic process [GO:1901605] Also known as: citrulline metabolism